{
  "term_label": "mitochondrion localization",
  "gene": "UniProtKB:O95140",
  "gene_name": "Mitofusin-2",
  "gene_symbol": "MFN2",
  "term_id": "GO:0051646"
}